{
  "gene": "UniProtKB:Q9H0N0",
  "term_label": "retrograde transport, endosome to Golgi",
  "gene_name": "Ras-related protein Rab-6C",
  "gene_symbol": "RAB6C",
  "term_id": "GO:0042147"
}